{
  "term_label": "immune response",
  "gene_symbol": "IGKV2-28",
  "term_id": "GO:0006955",
  "gene": "UniProtKB:A0A075B6P5",
  "gene_name": "Immunoglobulin kappa variable 2-28"
}